{
  "term_id": "UNKNOWN:0002",
  "term_label": "Unknown biological process",
  "gene": "UniProtKB:A0A075B6U9",
  "gene_name": "T cell receptor alpha joining 2 (non-functional) (Fragment)",
  "gene_symbol": "TRAJ2"
}